{
  "term_label": "G1/S transition of mitotic cell cycle",
  "gene": "UniProtKB:P46527",
  "gene_name": "Cyclin-dependent kinase inhibitor 1B",
  "term_id": "GO:0000082",
  "gene_symbol": "CDKN1B"
}